{
  "term_label": "Unknown molecular function",
  "gene_name": "Secernin-2",
  "gene_symbol": "SCRN2",
  "gene": "UniProtKB:Q96FV2",
  "term_id": "UNKNOWN:0001"
}